{
  "term_label": "potassium ion import across plasma membrane",
  "gene_symbol": "ATP4B",
  "gene_name": "Potassium-transporting ATPase subunit beta",
  "gene": "UniProtKB:P51164",
  "term_id": "GO:1990573"
}